{
  "gene_symbol": "HOXB4",
  "gene_name": "Homeobox protein Hox-B4",
  "gene": "UniProtKB:P17483",
  "term_id": "GO:0000978",
  "term_label": "RNA polymerase II cis-regulatory region sequence-specific DNA binding"
}